{
  "term_id": "GO:0006338",
  "gene_symbol": "ACTL6A",
  "gene_name": "Actin-like protein 6A",
  "gene": "UniProtKB:O96019",
  "term_label": "chromatin remodeling"
}